{
  "term_label": "regulation of postsynaptic membrane neurotransmitter receptor levels",
  "gene_symbol": "DLG1",
  "gene_name": "Disks large homolog 1",
  "term_id": "GO:0099072",
  "gene": "UniProtKB:Q12959"
}